{
  "gene_name": "PABIR family member 1",
  "term_label": "protein serine/threonine phosphatase inhibitor activity",
  "gene_symbol": "PABIR3",
  "gene": "UniProtKB:Q6P4D5",
  "term_id": "GO:0004865"
}